{
  "gene_symbol": "MAGEA4",
  "gene_name": "Melanoma-associated antigen 4",
  "term_id": "GO:0000122",
  "gene": "UniProtKB:P43358",
  "term_label": "negative regulation of transcription by RNA polymerase II"
}